meiotic DNA double-strand break processing involved in meiotic gene conversion [GO:0010704] (biological process) Definition: The cell cycle process in which the 5' to 3' exonucleolytic resection of the DNA at the site of the break to form a 3' single-strand DNA overhang resulting in the transfer of genetic information from one helix to another. Sources: GOC:dph, GOC:tb Relationships: is a type of meiotic DNA double-strand break processing [GO:0000706]; is part of meiotic gene conversion [GO:0006311]